{
  "gene_symbol": "IKBKB",
  "term_id": "GO:0004674",
  "gene_name": "Inhibitor of nuclear factor kappa-B kinase subunit beta",
  "gene": "UniProtKB:O14920",
  "term_label": "protein serine/threonine kinase activity"
}